nicotinate biosynthetic process [GO:1901849] (BP) Also known as: nicotinate anabolism, nicotinate biosynthesis, nicotinate formation, nicotinate synthesis Sources: GOC:TermGenie, GOC:yaf, UniPathway:UPA00830 Relationships: is a type of GO:0009821; is a type of monocarboxylic acid biosynthetic process [GO:0072330]; is a type of pyridine-containing compound biosynthetic process [GO:0072525]; is a type of GO:1901847 Definition: The chemical reactions and pathways resulting in the formation of nicotinate.